response to herbivore [GO:0080027] (biological process) Relationships: is a type of response to other organism [GO:0051707] References: PMID:18987211 Definition: Any process that results in a change in state or activity of a cell or an organism (in terms of movement, secretion, enzyme production, gene expression, etc.) as a result of a stimulus from a herbivore.